{
  "gene_symbol": "MIP",
  "term_id": "GO:0006833",
  "term_label": "water transport",
  "gene": "UniProtKB:P30301",
  "gene_name": "Lens fiber major intrinsic protein"
}